{
  "term_id": "GO:0005634",
  "gene": "UniProtKB:Q9UI95",
  "term_label": "nucleus",
  "gene_symbol": "MAD2L2",
  "gene_name": "Mitotic spindle assembly checkpoint protein MAD2B"
}